{
  "term_label": "paracellular tight junction channel activity",
  "gene": "UniProtKB:Q9Y5I7",
  "term_id": "GO:0160187",
  "gene_symbol": "CLDN16",
  "gene_name": "Claudin-16"
}